postsynaptic early endosome [GO:0098842] (cellular component) Note: Commonly used markers for postsynaptic early endosomes include RAB5A and EEA1. References: PMID:19603039, PMID:20820847, PMID:24727350 Definition: An early endosome of the postsynapse. It acts as the major sorting station on the endocytic pathway, targeting neurotransmitter receptors for degregation or recycling. Relationships: is a type of GO:0005769; is a type of postsynaptic endosome [GO:0098845]